{
  "gene": "UniProtKB:Q9Y651",
  "gene_symbol": "SOX21",
  "gene_name": "Transcription factor SOX-21",
  "term_label": "neuron differentiation",
  "term_id": "GO:0030182"
}